{
  "gene": "UniProtKB:P35626",
  "term_id": "GO:0001664",
  "gene_symbol": "GRK3",
  "gene_name": "Beta-adrenergic receptor kinase 2",
  "term_label": "G protein-coupled receptor binding"
}